nuclear pore cytoplasmic filaments [GO:0044614] (cellular component) Definition: Filamentous extensions on cytoplasmic face of the nuclear pore complex (NPC). In S. cerevisiae, Nup159p, Nup82p, and Nup42p contribute to the cytoplasmic filaments. In vertebrates, Nup358 is a major component. References: PMID:18046406, PMID:19524430, PMID:20947011, PMID:22419078 Sources: GOC:dgf Relationships: is a type of GO:0140513; is part of nuclear pore [GO:0005643] Also known as: cytoplasmic fibers of the NPC, cytoplasmic fibers of the nuclear pore complex